{
  "gene_name": "Kinesin-like protein KIF3C",
  "term_label": "microtubule motor activity",
  "gene_symbol": "KIF3C",
  "term_id": "GO:0003777",
  "gene": "UniProtKB:O14782"
}